{
  "gene_name": "Protein lifeguard 1",
  "term_id": "GO:1902042",
  "term_label": "negative regulation of extrinsic apoptotic signaling pathway via death domain receptors",
  "gene_symbol": "GRINA",
  "gene": "UniProtKB:Q7Z429"
}